{
  "gene_symbol": "GPR155",
  "gene_name": "Integral membrane protein GPR155",
  "gene": "UniProtKB:Q7Z3F1",
  "term_id": "UNKNOWN:0003",
  "term_label": "Unknown cellular component"
}